dADP binding [GO:0032563] (molecular function) Sources: GOC:mah Relationships: is a type of adenyl deoxyribonucleotide binding [GO:0032558]; is a type of anion binding [GO:0043168] Definition: Binding to dADP, deoxyadenosine diphosphate.